{
  "term_label": "extracellular matrix structural constituent",
  "gene_symbol": "ZAN",
  "term_id": "GO:0005201",
  "gene_name": "Zonadhesin",
  "gene": "UniProtKB:Q9Y493"
}